{
  "gene_name": "RUN domain-containing protein 3B",
  "gene": "UniProtKB:Q96NL0",
  "gene_symbol": "RUNDC3B",
  "term_id": "UNKNOWN:0003",
  "term_label": "Unknown cellular component"
}